{
  "gene_symbol": "HOXA3",
  "term_label": "RNA polymerase II cis-regulatory region sequence-specific DNA binding",
  "gene": "UniProtKB:O43365",
  "term_id": "GO:0000978",
  "gene_name": "Homeobox protein Hox-A3"
}